{
  "gene_name": "GTP cyclohydrolase 1 feedback regulatory protein",
  "term_label": "GTP cyclohydrolase binding",
  "term_id": "GO:0044549",
  "gene": "UniProtKB:P30047",
  "gene_symbol": "GCHFR"
}